{
  "gene_symbol": "ATG2A",
  "term_id": "GO:0032266",
  "gene_name": "Autophagy-related protein 2 homolog A",
  "term_label": "phosphatidylinositol-3-phosphate binding",
  "gene": "UniProtKB:Q2TAZ0"
}